{
  "gene": "UniProtKB:Q9H4F8",
  "gene_symbol": "SMOC1",
  "gene_name": "SPARC-related modular calcium-binding protein 1",
  "term_id": "GO:0005615",
  "term_label": "extracellular space"
}